cardiac blood vessel endothelial cell differentiation [GO:0060946] (biological process) Sources: GOC:mtg_heart Relationships: is a type of cardiac endothelial cell differentiation [GO:0003348]; is a type of blood vessel endothelial cell differentiation [GO:0060837] Definition: The process in which a relatively unspecialized cell acquires specialized features of a blood vessel endothelial cell of the heart. Blood vessel endothelial cells are thin flattened cells that line the inside surfaces of blood vessels.